regulation of NK T cell proliferation [GO:0051140] (biological process) Subtypes: negative regulation of NK T cell proliferation [GO:0051141], positive regulation of NK T cell proliferation [GO:0051142] References: PMID:12154375, PMID:9133426 Sources: ISBN:0781735149 Relationships: is_a GO:0046640; is a type of GO:0051133; regulates GO:0001866 Also known as: regulation of NK T lymphocyte proliferation, regulation of NK T-cell proliferation, regulation of NK T-lymphocyte proliferation, regulation of NKT cell proliferation, regulation of NT cell proliferation, regulation of natural T cell proliferation, regulation of natural killer T cell proliferation Definition: Any process that modulates the frequency, rate or extent of natural killer T cell proliferation.